negative regulation of ferricrocin biosynthetic process [GO:1900679] (biological process) Sources: GOC:TermGenie, GOC:di Relationships: is a type of regulation of ferricrocin biosynthetic process [GO:1900678]; is a type of GO:1905569; negatively regulates GO:0031171 Definition: Any process that stops, prevents or reduces the frequency, rate or extent of ferricrocin biosynthetic process. Also known as: down regulation of ferricrocin anabolism, down regulation of ferricrocin biosynthesis, down regulation of ferricrocin biosynthetic process, down regulation of ferricrocin formation, down regulation of ferricrocin synthesis, down-regulation of ferricrocin anabolism, down-regulation of ferricrocin biosynthesis, down-regulation of ferricrocin biosynthetic process, down-regulation of ferricrocin formation, down-regulation of ferricrocin synthesis, downregulation of ferricrocin anabolism, downregulation of ferricrocin biosynthesis, downregulation of ferricrocin biosynthetic process, downregulation of ferricrocin formation, downregulation of ferricrocin synthesis, inhibition of ferricrocin anabolism, inhibition of ferricrocin biosynthesis, inhibition of ferricrocin formation, inhibition of ferricrocin synthesis, negative regulation of ferricrocin anabolism, negative regulation of ferricrocin biosynthesis, negative regulation of ferricrocin formation, negative regulation of ferricrocin synthesis, down regulation of ferricrocin biosynthetic process, peptide formation, down regulation of ferricrocin biosynthetic process, peptide modification, down-regulation of ferricrocin biosynthetic process, peptide formation, down-regulation of ferricrocin biosynthetic process, peptide modification, downregulation of ferricrocin biosynthetic process, peptide formation, downregulation of ferricrocin biosynthetic process, peptide modification, inhibition of ferricrocin biosynthetic process, inhibition of ferricrocin biosynthetic process, peptide formation, inhibition of ferricrocin biosynthetic process, peptide modification, negative regulation of ferricrocin biosynthetic process, peptide formation, negative regulation of ferricrocin biosynthetic process, peptide modification